plant organ formation [GO:1905393] (biological process) Definition: The process that gives rise to the plant organ. This process pertains to the initial formation of a structure from unspecified parts. Sources: GOC:TermGenie, GOC:tb, GO_REF:0000081 Subtypes: lateral root formation [GO:0010311], leaf formation [GO:0010338], shoot axis formation [GO:0010346], bract formation [GO:0010434], floral organ formation [GO:0048449] Relationships: is a type of anatomical structure formation involved in morphogenesis [GO:0048646] Regulation: RO_0002211 by regulation of plant organ formation [GO:1905428]